{
  "term_id": "GO:0000800",
  "term_label": "lateral element",
  "gene_symbol": "SYCP2L",
  "gene": "UniProtKB:Q5T4T6",
  "gene_name": "Synaptonemal complex protein 2-like"
}